{
  "gene": "UniProtKB:Q8IY37",
  "term_id": "GO:0005730",
  "term_label": "nucleolus",
  "gene_symbol": "DHX37",
  "gene_name": "Probable ATP-dependent RNA helicase DHX37"
}